{
  "gene_symbol": "ANXA1",
  "gene": "UniProtKB:P04083",
  "term_label": "cytoplasm",
  "term_id": "GO:0005737",
  "gene_name": "Annexin A1"
}